mitochondrial inner membrane assembly complex [GO:1990677] (cellular component) References: PMID:24942160 Sources: GOC:bhm Also known as: inner membrane assembly complex, INAC complex, mitochondrion inner membrane assembly complex Relationships: is a type of inner mitochondrial membrane protein complex [GO:0098800] Definition: A protein complex that promotes the biogenesis of mitochondrial F1Fo-ATP synthase by facilitating assembly of the peripheral stalk. Loss of INAC function causes dissociation of the F1-domain from the membrane-integral Fo-portion. Note: An example of this is INA22 in Saccharomyces cerevisiae (P40576) in PMID:24942160 (inferred from direct assay/mutant phenotype/etc.).